{
  "gene": "UniProtKB:Q5W5W9",
  "gene_name": "Regulated endocrine-specific protein 18",
  "gene_symbol": "RESP18",
  "term_id": "UNKNOWN:0002",
  "term_label": "Unknown biological process"
}